PTEN phosphatase complex [GO:1990455] (cellular component) Note: An example of this is PTEN in human (P60484) in PMID:24766807 (inferred from direct assay). Relationships: is_a GO:1904144 Also known as: phosphatase and tensin homolog, phosphatase and tensin homolog deleted on chromosome ten homodimer, phosphatidylinositol 3,4,5-trisphosphate 3-phosphatase and dual-specificity protein phosphatase PTEN homodimer References: PMID:24766807 Sources: GOC:bhm Definition: A phospholipid phosphatase complex that catalyses the hydrolysis of the second messenger PtdIns (3,4,5)P3. Will also dephosphorylate PtdIns(3,4)P2, PtdIns3P, and Ins(1,3,4,5)P4. Dimerization is critical for its lipid phosphatase function.